{
  "term_label": "intracellular signal transduction",
  "gene_name": "MAP kinase-activated protein kinase 3",
  "term_id": "GO:0035556",
  "gene_symbol": "MAPKAPK3",
  "gene": "UniProtKB:Q16644"
}